{
  "gene_name": "Olfactory receptor 6C75",
  "gene_symbol": "OR6C75",
  "term_id": "UNKNOWN:0002",
  "term_label": "Unknown biological process",
  "gene": "UniProtKB:A6NL08"
}